negative regulation of receptor binding [GO:1900121] (biological process) Definition: Any process that stops, prevents or reduces the frequency, rate or extent of a protein or other molecule binding to a receptor. Sources: GOC:TermGenie, GOC:signaling Subtypes: negative regulation of cytokine activity [GO:0060302] Relationships: is a type of negative regulation of protein binding [GO:0032091]; is a type of regulation of receptor binding [GO:1900120]; negatively regulates signaling receptor binding [GO:0005102] Also known as: down regulation of receptor binding, down-regulation of receptor binding, downregulation of receptor binding, inhibition of receptor binding, inhibition of receptor ligand, down regulation of receptor-associated protein activity